{
  "term_label": "L-lactate dehydrogenase (NAD+) activity",
  "gene_name": "L-lactate dehydrogenase A-like 6B",
  "term_id": "GO:0004459",
  "gene": "UniProtKB:Q9BYZ2",
  "gene_symbol": "LDHAL6B"
}